{
  "term_label": "lysosome",
  "term_id": "GO:0005764",
  "gene": "UniProtKB:Q96S99",
  "gene_name": "Pleckstrin homology domain-containing family F member 1",
  "gene_symbol": "PLEKHF1"
}